{
  "gene": "UniProtKB:A1L4Q6",
  "gene_name": "Putative uncharacterized protein FLJ41423",
  "term_label": "Unknown biological process",
  "term_id": "UNKNOWN:0002",
  "gene_symbol": "A1L4Q6"
}